SAGA complex binding [GO:0062070] (molecular function) Definition: Binding to a SAGA complex. References: PMID:27185460 Relationships: is a type of protein-containing complex binding [GO:0044877]